{
  "gene_name": "Protein FAM200B",
  "gene": "UniProtKB:P0CF97",
  "gene_symbol": "FAM200B",
  "term_label": "Unknown biological process",
  "term_id": "UNKNOWN:0002"
}